regulation of membrane repolarization during action potential [GO:0098903] (biological process) Sources: GOC:dos, GOC:dph, GOC:tb, ISBN:978-0-07-139011-8 Subtypes: regulation of membrane repolarization during cardiac muscle cell action potential [GO:1905031] Relationships: is a type of regulation of membrane repolarization [GO:0060306]; is a type of GO:0098900; regulates membrane repolarization during action potential [GO:0086011] Definition: Any process that modulates the rate, frequency or extent of membrane repolarization during an action potential. Membrane repolarization is the process in which membrane potential changes in the repolarizing direction, towards the resting potential.